anaerobic lignin catabolic process [GO:1990487] (biological process) Also known as: anaerobic lignin degradation Relationships: is a type of lignin catabolic process [GO:0046274] Definition: The chemical reactions and pathways resulting in the breakdown of lignin in the absence of oxygen. Lignin is a class of polymers of phenylpropanoid units. Sources: DOI:10.1039/C3EE40932E, GOC:mengo_curators